{
  "gene": "UniProtKB:P48739",
  "gene_name": "Phosphatidylinositol transfer protein beta isoform",
  "term_id": "GO:0031210",
  "gene_symbol": "PITPNB",
  "term_label": "phosphatidylcholine binding"
}